{
  "gene": "UniProtKB:Q8N4B5",
  "gene_name": "Proline-rich protein 18",
  "term_id": "UNKNOWN:0003",
  "gene_symbol": "PRR18",
  "term_label": "Unknown cellular component"
}